{
  "gene_symbol": "DNAH9",
  "term_id": "GO:0051959",
  "gene": "UniProtKB:Q9NYC9",
  "gene_name": "Dynein axonemal heavy chain 9",
  "term_label": "dynein light intermediate chain binding"
}